macrolide metabolic process [GO:0033067] (biological process) Relationships: is_a antibiotic metabolic process [GO:0016999]; is a type of polyketide metabolic process [GO:0030638]; is a type of GO:1901334 Also known as: macrolide metabolism Definition: The chemical reactions and pathways involving macrolides, any of a large group of polyketide compounds that contain a large lactone ring with few or no double bonds and no nitrogen atoms, linked glycosidically to one or more sugar groups. The macrolides include the carbomycins, the erythromycins, oleandomycin, oligomycins, and the spiramycins, and act as antibiotics, mainly against Gram-positive bacteria. References: PMID:17298179 Sources: ISBN:0198506732 Subtypes: macrolide biosynthetic process [GO:0033068], enterobactin catabolic process [GO:0046214], GO:1901114